{
  "gene_symbol": "VSIR",
  "term_id": "GO:0005886",
  "gene": "UniProtKB:Q9H7M9",
  "gene_name": "V-type immunoglobulin domain-containing suppressor of T-cell activation",
  "term_label": "plasma membrane"
}